{
  "term_id": "GO:0002028",
  "gene": "UniProtKB:Q4KMZ8",
  "gene_symbol": "NKAIN1",
  "gene_name": "Sodium_potassium-transporting ATPase subunit beta-1-interacting protein 1",
  "term_label": "regulation of sodium ion transport"
}